{
  "term_label": "actin binding",
  "gene": "UniProtKB:P60673",
  "gene_name": "Profilin-3",
  "term_id": "GO:0003779",
  "gene_symbol": "PFN3"
}